negative regulation of cell communication by electrical coupling involved in cardiac conduction [GO:1901845] (BP) Definition: Any process that stops, prevents or reduces the frequency, rate or extent of cell communication by electrical coupling involved in cardiac conduction. Also known as: down regulation of cell communication by electrical coupling involved in cardiac conduction, down-regulation of cell communication by electrical coupling involved in cardiac conduction, downregulation of cell communication by electrical coupling involved in cardiac conduction, inhibition of cell communication by electrical coupling involved in cardiac conduction Relationships: is a type of negative regulation of cell communication by electrical coupling [GO:0010651]; is a type of GO:1901844; negatively regulates GO:0086064 References: PMID:17130302 Sources: GOC:BHF, GOC:TermGenie, GOC:rl